symbiont genome ejection through host cell envelope, contractile tail mechanism [GO:0099000] (biological process) Definition: Entry of a symbiont's genome into the host cell through the host cell envelope via a contractile tail ejection system consisting of a baseplate, a central tube and an external contractile sheath. Upon binding to the host cell surface, the baseplate changes its conformation and triggers sheath contraction, driving the rigid internal tail tube through the cell envelope. Occurs in non-enveloped prokaryotic viruses. References: PMID:26283379 Sources: GOC:dos, VZ:3950 Also known as: viral contractile tail ejection system, viral genome ejection through host cell envelope, contractile tail mechanism Relationships: is a type of symbiont genome ejection through host cell envelope [GO:0039678]